{
  "gene": "UniProtKB:P30520",
  "term_label": "IMP metabolic process",
  "gene_symbol": "ADSS2",
  "gene_name": "Adenylosuccinate synthetase isozyme 2",
  "term_id": "GO:0046040"
}